{
  "term_label": "Unknown cellular component",
  "gene_symbol": "GREP1",
  "gene": "UniProtKB:A0A0J9YXV3",
  "term_id": "UNKNOWN:0003",
  "gene_name": "Glycine-rich extracellular protein 1"
}